t-SNARE clustering [GO:1990656] (biological process) Relationships: is a type of GO:0072657 References: PMID:22528485 Regulation: regulated by regulation of t-SNARE clustering [GO:1904032]; negatively regulated by GO:1904033; RO_0002213 by GO:1904034 Definition: The clustering process in which t-SNARES are localized to distinct domains in the cell membrane. t-SNAREs are cell surface proteins which are part of secretory microdomain assemblies.